{
  "gene_name": "Putative protein FAM90A24P",
  "gene_symbol": "FAM90A24P",
  "gene": "UniProtKB:P0C7X0",
  "term_label": "Unknown biological process",
  "term_id": "UNKNOWN:0002"
}